{
  "gene_name": "Mediator of RNA polymerase II transcription subunit 8",
  "gene": "UniProtKB:Q96G25",
  "term_label": "transcription coregulator activity",
  "term_id": "GO:0003712",
  "gene_symbol": "MED8"
}